cellular response to chloramphenicol [GO:0072747] (biological process) Definition: Any process that results in a change in state or activity of a cell (in terms of movement, secretion, enzyme production, gene expression, etc.) as a result of a chloramphenicol stimulus. Relationships: is a type of response to chloramphenicol [GO:1901322]; is a type of cellular response to nitrogen compound [GO:1901699]; is a type of cellular response to oxygen-containing compound [GO:1901701] Sources: GOC:mah